{
  "gene_symbol": "MYO9A",
  "term_id": "GO:0005884",
  "term_label": "actin filament",
  "gene": "UniProtKB:B2RTY4",
  "gene_name": "Unconventional myosin-IXa"
}